{
  "gene_name": "CKLF-like MARVEL transmembrane domain-containing protein 3",
  "term_label": "membrane",
  "term_id": "GO:0016020",
  "gene_symbol": "CMTM3",
  "gene": "UniProtKB:Q96MX0"
}